{
  "gene_symbol": "TRABD2A",
  "term_label": "metalloendopeptidase activity",
  "term_id": "GO:0004222",
  "gene_name": "Metalloprotease TIKI1",
  "gene": "UniProtKB:Q86V40"
}